steroid Delta-isomerase activity [GO:0004769] (molecular function) Relationships: is_a intramolecular oxidoreductase activity, transposing C=C bonds [GO:0016863] Also known as: steroid D-isomerase activity, 3-oxosteroid delta5-delta4-isomerase activity, 3-oxosteroid isomerase activity, delta(5)-3-keto steroid isomerase activity, delta(5)-3-ketosteroid isomerase activity, delta(5)-3-oxosteroid isomerase activity, delta(5)-steroid isomerase activity, delta5(or delta4)-3-keto steroid isomerase activity, delta5-3-keto steroid isomerase activity, delta5-3-ketosteroid isomerase activity, delta5-3-oxosteroid isomerase activity, delta5-ketosteroid isomerase activity, delta5-steroid isomerase activity, hydroxysteroid isomerase activity, steroid isomerase activity Definition: Catalysis of the reaction: a 3-oxo-delta(5)-steroid = a 3-oxo-delta(4)-steroid. Sources: RHEA:14709